interleukin-37 production [GO:0150137] (BP) References: PMID:30362558 Sources: GOC:aruk Regulation: regulated by regulation of interleukin-37 production [GO:0150136]; negatively regulated by negative regulation of interleukin-37 production [GO:0150138]; positively regulated by GO:0150139 Also known as: interleukin-37 biosynthetic process Relationships: is a type of cytokine production [GO:0001816] Definition: The appearance of interleukin-37 due to biosynthesis or secretion following a cellular stimulus, resulting in an increase in its intracellular or extracellular levels.